{
  "gene_name": "Zinc finger protein 707",
  "term_label": "RNA polymerase II cis-regulatory region sequence-specific DNA binding",
  "gene": "UniProtKB:Q96C28",
  "gene_symbol": "ZNF707",
  "term_id": "GO:0000978"
}